positive regulation of meiosis I spindle assembly checkpoint [GO:1905326] (biological process) Also known as: up regulation of meiosis I spindle assembly checkpoint, up-regulation of meiosis I spindle assembly checkpoint, upregulation of meiosis I spindle assembly checkpoint, activation of meiosis I spindle assembly checkpoint Relationships: is a type of positive regulation of cell cycle process [GO:0090068]; is a type of positive regulation of spindle checkpoint [GO:0090232]; is a type of GO:1905325; is a type of positive regulation of reproductive process [GO:2000243]; positively regulates meiosis I spindle assembly checkpoint signaling [GO:1905318] References: PMID:26483559 Sources: GOC:TermGenie, GO_REF:0000058 Subtypes: activation of meiosis I spindle assembly checkpoint [GO:0090687] Definition: Any process that activates or increases the frequency, rate or extent of the meiosis I spindle assembly checkpoint.